photosynthetic state transition [GO:0062055] (biological process) Definition: A regulation of the phtosynthetic light reaction in which the light harvesting antenna complexes transition between photosystems. References: PMID:29967049 Relationships: is a type of GO:0042548